minor mitochondrial derivative [GO:0016009] (cellular component) Definition: The smaller of the two mitochondrial derivatives that arise by the unfolding of the Nebenkern during flagellum elongation. Relationships: is a type of mitochondrial derivative [GO:0016007] References: PMID:17123504, PMID:24211517, PMID:30802236 Sources: GOC:mah